{
  "gene_name": "Frizzled-6",
  "term_label": "canonical Wnt signaling pathway",
  "term_id": "GO:0060070",
  "gene": "UniProtKB:O60353",
  "gene_symbol": "FZD6"
}